{
  "gene": "UniProtKB:P02675",
  "gene_name": "Fibrinogen beta chain",
  "term_id": "GO:0070527",
  "gene_symbol": "FGB",
  "term_label": "platelet aggregation"
}